{
  "gene": "UniProtKB:Q96SQ9",
  "term_id": "GO:0008392",
  "gene_symbol": "CYP2S1",
  "gene_name": "Cytochrome P450 2S1",
  "term_label": "arachidonate epoxygenase activity"
}